regulation of branching involved in mammary gland duct morphogenesis [GO:0060762] (biological process) Definition: Any process that modulates the rate, frequency, or extent of branching involved in mammary gland duct morphogenesis. Sources: GOC:dph Subtypes: regulation of branching involved in mammary cord morphogenesis by fat precursor cell-epithelial cell signaling [GO:0060656] Relationships: is a type of regulation of morphogenesis of a branching structure [GO:0060688]; is a type of regulation of morphogenesis of an epithelium [GO:1905330]; is a type of GO:2000027; regulates GO:0060444